{
  "term_id": "GO:0033130",
  "gene_name": "Lymphocyte antigen 6E",
  "term_label": "acetylcholine receptor binding",
  "gene_symbol": "LY6E",
  "gene": "UniProtKB:Q16553"
}